fructose-2,6-bisphosphate 6-phosphatase activity [GO:0047386] (molecular function) Relationships: is_a GO:0050308 Sources: EC:3.1.3.54, RHEA:13333 Also known as: D-fructose-2,6-bisphosphate 6-phosphohydrolase activity, beta-D-fructose-2,6-bisphosphate 6-phosphohydrolase activity, fructose 2,6-bisphosphate-6-phosphohydrolase activity, fructose-2,6-bisphosphate 6-phosphohydrolase activity Definition: Catalysis of the reaction: beta-D-fructose 2,6-bisphosphate + H2O = beta-D-fructofuranose 2-phosphate + phosphate.